{
  "gene_name": "Histone deacetylase 11",
  "gene_symbol": "HDAC11",
  "term_label": "histone deacetylase activity",
  "term_id": "GO:0004407",
  "gene": "UniProtKB:Q96DB2"
}